{
  "term_id": "GO:0005886",
  "term_label": "plasma membrane",
  "gene": "UniProtKB:Q9H2J7",
  "gene_name": "Sodium-dependent neutral amino acid transporter B(0)AT2",
  "gene_symbol": "SLC6A15"
}